mitotic nuclear membrane reassembly [GO:0007084] (biological process) Definition: The mitotic cell cycle process involving ESCRTIII that results in reformation of the nuclear envelope after mitotic nuclear division. In organisms undergoing closed mitosis this involves resealing or 'repair' of the nuclear envelope in the nuclear bridge. Also known as: nuclear envelope repair, nuclear envelope resealing, mitotic nuclear envelope reassembly Relationships: is a type of nuclear membrane reassembly [GO:0031468]; is_a mitotic nuclear membrane organization [GO:0101024] References: PMID:26040712, PMID:28242692, PMID:32109380, PMID:32848252